{
  "gene_name": "Transcription factor PU.1",
  "term_id": "GO:0030154",
  "gene_symbol": "SPI1",
  "gene": "UniProtKB:P17947",
  "term_label": "cell differentiation"
}